negative regulation of stress-activated MAPK cascade [GO:0032873] (biological process) Subtypes: negative regulation of cell integrity MAPK cascade [GO:1903138] Also known as: down regulation of stress-activated MAPK cascade, down-regulation of stress-activated MAPK cascade, downregulation of stress-activated MAPK cascade, negative regulation of p38 MAPK signaling, negative regulation of p38 MAPK signalling, negative regulation of stress-activated MAPK signaling pathway, negative regulation of stress-activated MAPK signalling pathway, negative regulation of stress-activated MAPKKK cascade, negative regulation of stress-activated MAPKKK signaling pathway, negative regulation of stress-activated MAPKKK signalling pathway, inhibition of stress-activated MAPK cascade Relationships: is a type of regulation of stress-activated MAPK cascade [GO:0032872]; is a type of negative regulation of MAPK cascade [GO:0043409]; is a type of GO:0070303; negatively regulates stress-activated MAPK cascade [GO:0051403] Sources: GOC:mah Definition: Any process that stops, prevents, or reduces the frequency, rate or extent of signal transduction mediated by the stress-activated MAPK cascade.